{
  "term_label": "regulation of transcription by RNA polymerase II",
  "gene_name": "Transcriptional enhancer factor TEF-1",
  "term_id": "GO:0006357",
  "gene": "UniProtKB:P28347",
  "gene_symbol": "TEAD1"
}